{
  "gene": "UniProtKB:Q08554",
  "gene_symbol": "DSC1",
  "gene_name": "Desmocollin-1",
  "term_label": "desmosome",
  "term_id": "GO:0030057"
}